quinolinate catabolic process [GO:0034213] (biological process) Definition: The chemical reactions and pathways resulting in the breakdown of quinolinate, the anion of quinolinic acid, also known as 2,3-pyridinedicarboxylic acid. Sources: GOC:mah Relationships: is a type of dicarboxylic acid catabolic process [GO:0043649]; is a type of quinolinate metabolic process [GO:0046874]; is_a pyridine-containing compound catabolic process [GO:0072526] Also known as: quinolinate breakdown, quinolinate catabolism, quinolinate degradation